{
  "term_label": "Unknown cellular component",
  "term_id": "UNKNOWN:0003",
  "gene_symbol": "OR5J2",
  "gene_name": "Olfactory receptor 5J2",
  "gene": "UniProtKB:Q8NH18"
}